pyroptosome complex assembly [GO:1904270] (biological process) Relationships: is a type of protein-containing complex assembly [GO:0065003] References: PMID:17964261 Sources: GOC:TermGenie, GO_REF:0000079 Also known as: ASC pyroptosome assembly, ASC pyroptosome formation, pyroptosome complex formation Definition: The aggregation, arrangement and bonding together of a set of components to form a pyroptosome complex.